{
  "gene_name": "GDP-Man:Man(3)GlcNAc(2)-PP-Dol alpha-1,2-mannosyltransferase",
  "gene_symbol": "ALG11",
  "term_label": "endoplasmic reticulum membrane",
  "term_id": "GO:0005789",
  "gene": "UniProtKB:Q2TAA5"
}